{
  "gene_name": "WASH complex subunit 3",
  "gene_symbol": "WASHC3",
  "term_id": "GO:0006887",
  "term_label": "exocytosis",
  "gene": "UniProtKB:Q9Y3C0"
}